{
  "gene": "UniProtKB:Q9H2D6",
  "term_id": "GO:1900026",
  "gene_name": "TRIO and F-actin-binding protein",
  "gene_symbol": "TRIOBP",
  "term_label": "positive regulation of substrate adhesion-dependent cell spreading"
}